{
  "gene_symbol": "SH2B3",
  "gene_name": "SH2B adapter protein 3",
  "term_id": "GO:0035556",
  "gene": "UniProtKB:Q9UQQ2",
  "term_label": "intracellular signal transduction"
}